{
  "term_label": "peroxisomal membrane",
  "gene_symbol": "ABCD2",
  "gene_name": "ATP-binding cassette sub-family D member 2",
  "gene": "UniProtKB:Q9UBJ2",
  "term_id": "GO:0005778"
}